{
  "gene_name": "5'-AMP-activated protein kinase subunit gamma-3",
  "gene": "UniProtKB:Q9UGI9",
  "term_label": "nucleotide-activated protein kinase complex",
  "term_id": "GO:0031588",
  "gene_symbol": "PRKAG3"
}